positive regulation of smooth muscle cell proliferation [GO:0048661] (biological process) Definition: Any process that activates or increases the rate or extent of smooth muscle cell proliferation. Sources: CL:0000192, GOC:ebc Also known as: positive regulation of SMC proliferation, up regulation of smooth muscle cell proliferation, up-regulation of smooth muscle cell proliferation, upregulation of smooth muscle cell proliferation, activation of smooth muscle cell proliferation, stimulation of smooth muscle cell proliferation Relationships: is a type of GO:0008284; is a type of GO:0048660; positively regulates smooth muscle cell proliferation [GO:0048659] Subtypes: GO:1904707